{
  "gene_symbol": "TM2D2",
  "gene": "UniProtKB:Q9BX73",
  "gene_name": "TM2 domain-containing protein 2",
  "term_label": "Unknown molecular function",
  "term_id": "UNKNOWN:0001"
}